{
  "term_label": "chloride transmembrane transport",
  "gene_symbol": "GABRG1",
  "gene_name": "Gamma-aminobutyric acid receptor subunit gamma-1",
  "gene": "UniProtKB:Q8N1C3",
  "term_id": "GO:1902476"
}